{
  "term_id": "GO:0050839",
  "gene_symbol": "TJP2",
  "gene": "UniProtKB:Q9UDY2",
  "gene_name": "Tight junction protein ZO-2",
  "term_label": "cell adhesion molecule binding"
}